{
  "gene_name": "Ketimine reductase mu-crystallin",
  "gene_symbol": "CRYM",
  "gene": "UniProtKB:Q14894",
  "term_label": "cytoplasm",
  "term_id": "GO:0005737"
}